positive regulation of nematode pharyngeal pumping [GO:1903746] (biological process) References: PMID:25329901 Sources: GOC:TermGenie, GOC:kmv, GO_REF:0000058 Definition: Any process that activates or increases the frequency, rate or extent of nematode pharyngeal pumping. Also known as: up regulation of pharyngeal pumping, up-regulation of pharyngeal pumping, upregulation of pharyngeal pumping, activation of pharyngeal pumping, activation of pumping behavior, positive regulation of pumping behavior, up regulation of pumping behavior, up-regulation of pumping behavior, upregulation of pumping behavior Relationships: is a type of regulation of nematode pharyngeal pumping [GO:0043051]; is a type of positive regulation of eating behavior [GO:1904000]; positively regulates nematode pharyngeal pumping [GO:0043050]